{
  "term_label": "synapse",
  "gene": "UniProtKB:Q8WXA8",
  "term_id": "GO:0045202",
  "gene_name": "5-hydroxytryptamine receptor 3C",
  "gene_symbol": "HTR3C"
}